{
  "gene_name": "Scavenger receptor class A member 3",
  "term_id": "UNKNOWN:0003",
  "term_label": "Unknown cellular component",
  "gene": "UniProtKB:Q6AZY7",
  "gene_symbol": "SCARA3"
}